{
  "gene": "UniProtKB:P98161",
  "gene_symbol": "PKD1",
  "term_label": "plasma membrane",
  "gene_name": "Polycystin-1",
  "term_id": "GO:0005886"
}